{
  "term_id": "GO:0006357",
  "gene_symbol": "ZKSCAN7",
  "gene_name": "Zinc finger protein with KRAB and SCAN domains 7",
  "term_label": "regulation of transcription by RNA polymerase II",
  "gene": "UniProtKB:Q9P0L1"
}